{
  "term_id": "GO:0000288",
  "gene_symbol": "PDE12",
  "term_label": "nuclear-transcribed mRNA catabolic process, deadenylation-dependent decay",
  "gene_name": "2',5'-phosphodiesterase 12",
  "gene": "UniProtKB:Q6L8Q7"
}